{
  "term_id": "GO:0048471",
  "gene_name": "Protein S100-A6",
  "term_label": "perinuclear region of cytoplasm",
  "gene_symbol": "S100A6",
  "gene": "UniProtKB:P06703"
}